{
  "gene": "UniProtKB:Q9BVK6",
  "gene_symbol": "TMED9",
  "gene_name": "Transmembrane emp24 domain-containing protein 9",
  "term_id": "GO:0005794",
  "term_label": "Golgi apparatus"
}